{
  "gene_name": "Pseudouridylate synthase 7 homolog",
  "term_label": "pseudouridine synthesis",
  "gene_symbol": "PUS7",
  "gene": "UniProtKB:Q96PZ0",
  "term_id": "GO:0001522"
}